{
  "term_label": "Unknown biological process",
  "gene_symbol": "CCDC51",
  "term_id": "UNKNOWN:0002",
  "gene": "UniProtKB:Q96ER9",
  "gene_name": "Mitochondrial potassium channel"
}